{
  "gene_symbol": "NUMA1",
  "gene": "UniProtKB:Q14980",
  "term_label": "mitotic spindle pole",
  "gene_name": "Nuclear mitotic apparatus protein 1",
  "term_id": "GO:0097431"
}